{
  "gene_symbol": "CYP11A1",
  "gene": "UniProtKB:P05108",
  "term_id": "GO:0006700",
  "gene_name": "Cholesterol side-chain cleavage enzyme, mitochondrial",
  "term_label": "C21-steroid hormone biosynthetic process"
}